{
  "term_id": "GO:0005634",
  "gene": "UniProtKB:Q99612",
  "gene_symbol": "KLF6",
  "gene_name": "Krueppel-like factor 6",
  "term_label": "nucleus"
}